{
  "gene": "UniProtKB:P81534",
  "gene_name": "Beta-defensin 103",
  "gene_symbol": "DEFB103B",
  "term_id": "GO:0042056",
  "term_label": "chemoattractant activity"
}